regulation of triglyceride metabolic process [GO:0090207] (biological process) Relationships: is a type of regulation of lipid metabolic process [GO:0019216]; regulates triglyceride metabolic process [GO:0006641] Sources: GOC:dph, GOC:sl, GOC:tb Subtypes: regulation of triglyceride biosynthetic process [GO:0010866], regulation of triglyceride catabolic process [GO:0010896], positive regulation of triglyceride metabolic process [GO:0090208], negative regulation of triglyceride metabolic process [GO:0090209] Definition: Any process that modulates the frequency, rate or extent of the chemical reactions and pathways involving triglyceride, any triester of glycerol.